glyoxylate catabolic process [GO:0009436] (BP) Relationships: is a type of aldehyde catabolic process [GO:0046185]; is a type of GO:0046487; is a type of monocarboxylic acid catabolic process [GO:0072329] Sources: ISBN:0198506732 Definition: The chemical reactions and pathways resulting in the breakdown of glyoxylate, the anion of glyoxylic acid, HOC-COOH. Also known as: glyoxylate breakdown, glyoxylate catabolism, glyoxylate degradation